positive regulation of DNA-templated transcription [GO:0045893] (BP) Sources: GOC:go_curators, GOC:txnOH Subtypes: positive regulation of DNA-templated transcription, elongation [GO:0032786], positive regulation of mating-type specific transcription, DNA-templated [GO:0045895], positive regulation of transcription by RNA polymerase I [GO:0045943], GO:0045944, positive regulation of transcription by RNA polymerase III [GO:0045945], carbon catabolite activation of transcription [GO:0045991], positive regulation of antisense RNA transcription [GO:0060196], positive regulation of termination of DNA-templated transcription [GO:0060566], positive regulation of transcription from a mobile element promoter [GO:0061435], positive regulation of transcription by transcription factor localization [GO:0061586], nitrogen catabolite activation of transcription [GO:0090294], positive regulation of piRNA transcription [GO:0140543], positive regulation of miRNA transcription [GO:1902895], positive regulation of mitochondrial transcription [GO:1903109], GO:1904281, positive regulation of DNA-templated transcription initiation [GO:2000144] Definition: Any process that activates or increases the frequency, rate or extent of cellular DNA-templated transcription. Relationships: is_a regulation of DNA-templated transcription [GO:0006355]; is a type of positive regulation of RNA biosynthetic process [GO:1902680]; positively regulates DNA-templated transcription [GO:0006351] Also known as: positive regulation of cellular transcription, DNA-dependent, positive regulation of transcription, DNA-dependent, positive regulation of transcription, DNA-templated, up regulation of transcription, DNA-dependent, up-regulation of transcription, DNA-dependent, upregulation of transcription, DNA-dependent, activation of transcription, DNA-dependent, stimulation of gene-specific transcription, stimulation of transcription, DNA-dependent, activation of gene-specific transcription, positive regulation of gene-specific transcription, transcription activator activity, up regulation of gene-specific transcription, up-regulation of gene-specific transcription, upregulation of gene-specific transcription